{
  "gene_symbol": "RPS10",
  "term_id": "UNKNOWN:0002",
  "gene": "UniProtKB:P46783",
  "gene_name": "Small ribosomal subunit protein eS10",
  "term_label": "Unknown biological process"
}